{
  "term_label": "very long-chain fatty acid biosynthetic process",
  "gene": "UniProtKB:A1L3X0",
  "gene_symbol": "ELOVL7",
  "gene_name": "Elongation of very long chain fatty acids protein 7",
  "term_id": "GO:0042761"
}